TOC-TIC supercomplex I [GO:0061927] (cellular component) References: PMID:28745032 Relationships: is a type of protein-containing complex [GO:0032991]; is part of chloroplast [GO:0009507] Definition: The protein transport macromolecular complex of the chloroplast membrane that interacts with the precursor proteins and contains components of both the outer membrane and inner membrane complexes containing at least Toc75, Toc159, Toc34 and Tic110.